vein smooth muscle contraction [GO:0014826] (biological process) Relationships: is a type of phasic smooth muscle contraction [GO:0014821]; is a type of vascular associated smooth muscle contraction [GO:0014829] Sources: GOC:mtg_muscle, MA:0000715, MSH:D014680 Definition: A process in which force is generated within smooth muscle tissue, resulting in a change in muscle geometry. This process occurs in the vein. Force generation involves a chemo-mechanical energy conversion step that is carried out by the actin/myosin complex activity, which generates force through ATP hydrolysis. The vein is a vessel carrying blood away from the capillary beds. Regulation: regulated by GO:0062086; RO_0002213 by positive regulation of vein smooth muscle contraction [GO:0062087]; negatively regulated by GO:0062088